{
  "term_label": "membrane",
  "gene": "UniProtKB:Q9BXB5",
  "gene_symbol": "OSBPL10",
  "term_id": "GO:0016020",
  "gene_name": "Oxysterol-binding protein-related protein 10"
}